{
  "gene_symbol": "HNRNPUL1",
  "term_id": "GO:0000380",
  "term_label": "alternative mRNA splicing, via spliceosome",
  "gene": "UniProtKB:Q9BUJ2",
  "gene_name": "Heterogeneous nuclear ribonucleoprotein U-like protein 1"
}